{
  "gene": "UniProtKB:B6A8C7",
  "gene_name": "T-cell-interacting, activating receptor on myeloid cells protein 1",
  "term_id": "GO:0004888",
  "term_label": "transmembrane signaling receptor activity",
  "gene_symbol": "TARM1"
}